{
  "term_id": "GO:0000978",
  "term_label": "RNA polymerase II cis-regulatory region sequence-specific DNA binding",
  "gene_symbol": "IRF5",
  "gene_name": "Interferon regulatory factor 5",
  "gene": "UniProtKB:Q13568"
}